mitotic cytokinesis, division site positioning [GO:1902408] (biological process) Definition: The process in which a contractile ring is positioned in a specific location during the mitotic cell cycle. This process is critical for both for both symmetric and asymmetric cell divisions. References: PMID:26553932, PMID:28162898 Also known as: mitotic cytokinesis, site selection Relationships: is a type of cytokinesis, division site positioning [GO:0007105]; is a type of mitotic cytokinetic process [GO:1902410] Regulation: regulated by regulation of mitotic cytokinesis, division site positioning [GO:1902472]; positively regulated by GO:1903617